{
  "gene_name": "Myeloid-associated differentiation marker",
  "term_id": "UNKNOWN:0001",
  "gene_symbol": "MYADM",
  "term_label": "Unknown molecular function",
  "gene": "UniProtKB:Q96S97"
}